{
  "gene_name": "Cathepsin G",
  "term_id": "GO:0005615",
  "gene": "UniProtKB:P08311",
  "gene_symbol": "CTSG",
  "term_label": "extracellular space"
}